{
  "gene": "UniProtKB:A0A2R8YEH3",
  "term_label": "detection of chemical stimulus involved in sensory perception of smell",
  "gene_symbol": "LOC112268384",
  "gene_name": "Olfactory receptor",
  "term_id": "GO:0050911"
}